{
  "gene": "UniProtKB:Q96GX2",
  "term_label": "Unknown cellular component",
  "gene_symbol": "ATXN7L3B",
  "gene_name": "Ataxin-7-like protein 3B",
  "term_id": "UNKNOWN:0003"
}